{
  "gene_symbol": "TSPAN32",
  "gene_name": "Tetraspanin-32",
  "term_id": "UNKNOWN:0001",
  "gene": "UniProtKB:Q96QS1",
  "term_label": "Unknown molecular function"
}